cyanelle [GO:0009842] (cellular component) Relationships: is a type of plastid [GO:0009536] Definition: A plastid that contains unstacked, phycobilisome-bearing thylakoid membranes and is surrounded by a double membrane with a peptidoglycan layer in the intermembrane space between the two envelope membranes. Cyanelles are characteristic of algae in the class Glaucophyta, and may represent an ancestral form of plastid. Sources: ISBN:0521316871, ISBN:1402001894 Also known as: cyanoplast, muroplast